circadian regulation of translation [GO:0097167] (biological process) Definition: Any process that modulates the frequency, rate or extent of mRNA translation with a regularity of approximately 24 hours. References: PMID:17264215 Sources: GOC:ans Also known as: regulation of mRNA translation in response to circadian clock Relationships: is a type of regulation of translation [GO:0006417]; is a type of circadian rhythm [GO:0007623]